DNA-(apurinic or apyrimidinic site) endonuclease activity [GO:0003906] (molecular function) Also known as: UV endonuclease, AP deoxyendoribonuclease activity, abasic deoxyendoribonuclease activity, apurinic deoxyendoribonuclease activity, apurinic/apyrimidinic endodeoxyribonuclease activity, apyrimidinic deoxyendoribonuclease activity, deoxyribonuclease (apurinic or apyrimidinic) activity, endonuclease VIII activity Relationships: is a type of DNA endonuclease activity [GO:0004520] Subtypes: class II DNA-(apurinic or apyrimidinic site) endonuclease activity [GO:0052720], class I DNA-(apurinic or apyrimidinic site) endonuclease activity [GO:0140078] Definition: Catalysis of the cleavage of the C-O-P bond in the AP site created when DNA glycosylase removes a damaged base, involved in the DNA base excision repair pathway (BER). Sources: Wikipedia:AP_endonuclease